positive regulation of adiponectin secretion [GO:0070165] (biological process) Definition: Any process that activates or increases the frequency, rate or extent of the regulated release of adiponectin from a cell. Relationships: is a type of positive regulation of hormone secretion [GO:0046887]; is a type of positive regulation of protein secretion [GO:0050714]; is a type of positive regulation of multicellular organismal process [GO:0051240]; is a type of regulation of adiponectin secretion [GO:0070163]; positively regulates adiponectin secretion [GO:0070162] Also known as: up regulation of adiponectin secretion, up-regulation of adiponectin secretion, upregulation of adiponectin secretion, activation of adiponectin secretion, stimulation of adiponectin secretion Sources: GOC:BHF, GOC:mah